{
  "gene": "UniProtKB:Q96RT7",
  "term_label": "gamma-tubulin complex",
  "gene_name": "Gamma-tubulin complex component 6",
  "gene_symbol": "TUBGCP6",
  "term_id": "GO:0000930"
}